azole:proton antiporter activity [GO:0045119] (molecular function) Sources: GOC:ai, ISBN:3527307206, Wikipedia:Azole Definition: Enables the transfer of a solute or solutes from one side of a membrane to the other according to the reaction: H+(out) + azole(in) = H+(in) + azole(out). Azoles are heterocyclic compounds found in many biologically important substances. Subtypes: fluconazole:proton antiporter activity [GO:0015313], aminotriazole:proton antiporter activity [GO:0015314], L-histidine, sodium:proton antiporter activity [GO:0140832] Also known as: azole:hydrogen antiporter activity, bicyclomycin/sulfathiazole:hydrogen antiporter activity Relationships: is_a proton transmembrane transporter activity [GO:0015078]; is a type of antiporter activity [GO:0015297]; is a type of azole transmembrane transporter activity [GO:1901474]